{
  "gene": "UniProtKB:P55072",
  "gene_symbol": "VCP",
  "gene_name": "Transitional endoplasmic reticulum ATPase",
  "term_label": "proteasome-mediated ubiquitin-dependent protein catabolic process",
  "term_id": "GO:0043161"
}